{
  "gene": "UniProtKB:O94933",
  "gene_symbol": "SLITRK3",
  "gene_name": "SLIT and NTRK-like protein 3",
  "term_id": "GO:0007409",
  "term_label": "axonogenesis"
}